{
  "gene_symbol": "MYBPC1",
  "term_id": "GO:0045214",
  "gene_name": "Myosin-binding protein C, slow-type",
  "term_label": "sarcomere organization",
  "gene": "UniProtKB:Q00872"
}